galactitol-1-phosphate 5-dehydrogenase activity [GO:0008868] (molecular function) Definition: Catalysis of the reaction: galactitol-1-phosphate + NAD+ = D-tagatose 6-phosphate + NADH + H+. Relationships: is a type of GO:0016616 Sources: EC:1.1.1.251 Also known as: galactitol-1-phosphate:NAD+ oxidoreductase activity